omega peptidase activity [GO:0008242] (molecular function) Relationships: is a type of GO:0008233 References: PMID:20157488, PMID:9920379 Sources: EC:3.4.19.- Also known as: peptidase activity, acting on peptides containing modified amino acids Definition: Catalysis of the cleavage of non-standard peptide bonds releasing substituted amino acids such as pyroglutamate or cleave isopeptide bonds, such as many deubiquitinating enzymes. Subtypes: leukotriene-C(4) hydrolase [GO:0002951], beta-aspartyl-peptidase activity [GO:0008798], pyroglutamyl-peptidase activity [GO:0016920], gamma-glutamyl-peptidase activity [GO:0034722], glutathione hydrolase activity [GO:0036374]